vesicle localization [GO:0051648] (biological process) Relationships: is a type of organelle localization [GO:0051640] Also known as: cytoplasmic vesicle localization, establishment and maintenance of vesicle localization, vesicle localisation Definition: Any process in which a vesicle or vesicles are transported to, and/or maintained in, a specific location. Subtypes: GO:0032252, establishment of vesicle localization [GO:0051650], maintenance of vesicle location [GO:0051655], pigment granule localization [GO:0051875], synaptic vesicle localization [GO:0097479], contractile vacuole localization [GO:0140027] Sources: GOC:ai